{
  "gene_name": "Tyrosine-protein kinase Fgr",
  "gene_symbol": "FGR",
  "term_id": "GO:0004715",
  "gene": "UniProtKB:P09769",
  "term_label": "non-membrane spanning protein tyrosine kinase activity"
}